{
  "term_id": "GO:0031966",
  "gene_symbol": "SDHB",
  "term_label": "mitochondrial membrane",
  "gene_name": "Succinate dehydrogenase [ubiquinone] iron-sulfur subunit, mitochondrial",
  "gene": "UniProtKB:P21912"
}